tissue morphogenesis [GO:0048729] (biological process) Definition: The process in which the anatomical structures of a tissue are generated and organized. Sources: GOC:dph, GOC:jid Relationships: is a type of GO:0009653; is part of GO:0009888 Subtypes: morphogenesis of an epithelium [GO:0002009], GO:0003404, ectodermal digestive tract development [GO:0007439], floor plate morphogenesis [GO:0033505], dorsal closure, amnioserosa morphology change [GO:0046664], mesoderm morphogenesis [GO:0048332], GO:0060415, cartilage morphogenesis [GO:0060536], Peyer's patch morphogenesis [GO:0061146], ganglion morphogenesis [GO:0061552], renal capsule morphogenesis [GO:0072128], mesenchyme morphogenesis [GO:0072132], fibrous ring of heart morphogenesis [GO:1905285]